{
  "gene_symbol": "ADH1A",
  "term_id": "GO:0008270",
  "gene": "UniProtKB:P07327",
  "gene_name": "Alcohol dehydrogenase 1A",
  "term_label": "zinc ion binding"
}